{
  "term_id": "GO:0010572",
  "gene": "UniProtKB:P40197",
  "gene_symbol": "GP5",
  "gene_name": "Platelet glycoprotein V",
  "term_label": "positive regulation of platelet activation"
}